{
  "gene_name": "Neurocan core protein",
  "term_id": "GO:0045202",
  "gene": "UniProtKB:O14594",
  "gene_symbol": "NCAN",
  "term_label": "synapse"
}